{
  "gene": "UniProtKB:Q86UB2",
  "term_label": "single-stranded DNA binding",
  "gene_name": "Basic immunoglobulin-like variable motif-containing protein",
  "term_id": "GO:0003697",
  "gene_symbol": "BIVM"
}